{
  "gene_name": "Acyl-coenzyme A synthetase ACSM2B, mitochondrial",
  "term_id": "GO:0005759",
  "gene_symbol": "ACSM2B",
  "term_label": "mitochondrial matrix",
  "gene": "UniProtKB:Q68CK6"
}